{
  "term_id": "UNKNOWN:0001",
  "term_label": "Unknown molecular function",
  "gene": "UniProtKB:Q969E2",
  "gene_symbol": "SCAMP4",
  "gene_name": "Secretory carrier-associated membrane protein 4"
}